{
  "gene_name": "Beclin-2",
  "term_label": "phosphatidylinositol 3-kinase complex, class III, type I",
  "term_id": "GO:0034271",
  "gene_symbol": "BECN2",
  "gene": "UniProtKB:A8MW95"
}